positive regulation of CD4-positive, CD25-positive, alpha-beta regulatory T cell differentiation involved in immune response [GO:0032834] (biological process) Definition: Any process that activates or increases the frequency, rate or extent of differentiation of CD4-positive, CD25-positive, alpha-beta regulatory T cells as part of an immune response. Sources: GOC:mah Also known as: activation of CD4-positive, CD25-positive, alpha-beta regulatory T cell differentiation during immune response, stimulation of CD4-positive, CD25-positive, alpha-beta regulatory T cell differentiation during immune response, positive regulation of CD4-positive, CD25-positive, alpha-beta regulatory T cell development involved in immune response, positive regulation of CD4-positive, CD25-positive, alpha-beta regulatory T cell differentiation during immune response, positive regulation of CD4-positive, CD25-positive, alpha-beta regulatory T lymphocyte differentiation during immune response, positive regulation of CD4-positive, CD25-positive, alpha-beta regulatory T-cell differentiation during immune response, positive regulation of CD4-positive, CD25-positive, alpha-beta regulatory T-lymphocyte differentiation during immune response, up regulation of CD4-positive, CD25-positive, alpha-beta regulatory T cell differentiation during immune response, up-regulation of CD4-positive, CD25-positive, alpha-beta regulatory T cell differentiation during immune response, upregulation of CD4-positive, CD25-positive, alpha-beta regulatory T cell differentiation during immune response Note: Note that immunologists typically use the word 'development' to refer to cells of B or T cell lineages undergoing the process that GO describes as 'cell differentiation'. Relationships: is_a positive regulation of immune effector process [GO:0002699]; is a type of positive regulation of CD4-positive, CD25-positive, alpha-beta regulatory T cell differentiation [GO:0032831]; is a type of regulation of CD4-positive, CD25-positive, alpha-beta regulatory T cell differentiation involved in immune response [GO:0032832]; is a type of positive regulation of immune response [GO:0050778]; positively regulates CD4-positive, CD25-positive, alpha-beta regulatory T cell differentiation involved in immune response [GO:0002298]